monoferuloyl di-(hydroxyferuloyl) spermidine meta-hydroxylase activity [GO:0072552] (molecular function) Relationships: is a type of tri-(feruloyl or hydroxyferuloyl) spermidine meta-hydroxylase activity [GO:0072532] Definition: Catalysis of the reaction: monoferuloyl di-(hydroxyferuloyl) spermidine + NADPH + O2 = tri-(hydroxyferuloyl) spermidine + NADP+ + H2O. References: PMID:19779199 Sources: GOC:kad